negative regulation of metaphase/anaphase transition of cell cycle [GO:1902100] (biological process) Relationships: is_a GO:1901988; is a type of regulation of metaphase/anaphase transition of cell cycle [GO:1902099]; negatively regulates GO:0044784 Sources: GOC:TermGenie, GOC:mtg_cell_cycle Definition: Any process that stops, prevents or reduces the frequency, rate or extent of metaphase/anaphase transition of cell cycle. Subtypes: GO:0045841, negative regulation of metaphase/anaphase transition of meiotic cell cycle [GO:1902103] Also known as: down regulation of metaphase/anaphase transition of cell cycle, down-regulation of metaphase/anaphase transition of cell cycle, downregulation of metaphase/anaphase transition of cell cycle, inhibition of metaphase/anaphase transition of cell cycle